{
  "gene_name": "Chromodomain-helicase-DNA-binding protein 5",
  "term_id": "GO:0000785",
  "gene": "UniProtKB:Q8TDI0",
  "gene_symbol": "CHD5",
  "term_label": "chromatin"
}